{
  "term_id": "GO:0060396",
  "gene": "UniProtKB:P15509",
  "gene_symbol": "CSF2RA",
  "gene_name": "Granulocyte-macrophage colony-stimulating factor receptor subunit alpha",
  "term_label": "growth hormone receptor signaling pathway"
}